{
  "gene_name": "Inorganic pyrophosphatase 2, mitochondrial",
  "gene": "UniProtKB:Q9H2U2",
  "term_id": "GO:0004427",
  "term_label": "inorganic diphosphate phosphatase activity",
  "gene_symbol": "PPA2"
}